{
  "gene": "UniProtKB:Q96BR5",
  "term_label": "protein-disulfide reductase activity",
  "gene_name": "Cytochrome c oxidase assembly factor 7",
  "gene_symbol": "COA7",
  "term_id": "GO:0015035"
}